{
  "gene": "UniProtKB:A0A7P0TAN4",
  "gene_symbol": "LOC122539214",
  "term_label": "nucleus",
  "gene_name": "Uncharacterized protein",
  "term_id": "GO:0005634"
}